{
  "term_id": "GO:0006357",
  "term_label": "regulation of transcription by RNA polymerase II",
  "gene_symbol": "TBX6",
  "gene_name": "T-box transcription factor TBX6",
  "gene": "UniProtKB:O95947"
}